{
  "gene": "UniProtKB:P0CG12",
  "term_id": "UNKNOWN:0001",
  "gene_name": "Decreased expression in renal and prostate cancer protein",
  "gene_symbol": "DERPC",
  "term_label": "Unknown molecular function"
}